{
  "gene": "UniProtKB:O95433",
  "term_label": "cytosol",
  "term_id": "GO:0005829",
  "gene_name": "Activator of 90 kDa heat shock protein ATPase homolog 1",
  "gene_symbol": "AHSA1"
}